sugar transmembrane transporter activity [GO:0051119] (molecular function) Definition: Enables the transfer of a sugar from one side of a membrane to the other. A sugar is any member of a class of sweet, water-soluble, crystallizable carbohydrates, which are the monosaccharides and smaller oligosaccharides. Sources: GOC:ai, GOC:mtg_transport, ISBN:0815340729 Subtypes: monosaccharide transmembrane transporter activity [GO:0015145] Also known as: sugar/polyol channel activity Relationships: is a type of carbohydrate transmembrane transporter activity [GO:0015144]